{
  "term_label": "nucleotide-activated protein kinase complex",
  "gene_symbol": "PRKAB1",
  "term_id": "GO:0031588",
  "gene": "UniProtKB:Q9Y478",
  "gene_name": "5'-AMP-activated protein kinase subunit beta-1"
}